{
  "term_label": "Unknown molecular function",
  "gene_name": "Eukaryotic translation elongation factor 1 epsilon-1",
  "term_id": "UNKNOWN:0001",
  "gene": "UniProtKB:O43324",
  "gene_symbol": "EEF1E1"
}